{
  "gene": "UniProtKB:P50583",
  "term_label": "Unknown cellular component",
  "term_id": "UNKNOWN:0003",
  "gene_name": "Bis(5'-nucleosyl)-tetraphosphatase [asymmetrical]",
  "gene_symbol": "NUDT2"
}